{
  "term_id": "GO:0002486",
  "gene_symbol": "HLA-G",
  "gene": "UniProtKB:P17693",
  "gene_name": "HLA class I histocompatibility antigen, alpha chain G",
  "term_label": "antigen processing and presentation of endogenous peptide antigen via MHC class I via ER pathway, TAP-independent"
}